{
  "gene_name": "Putative ribosomal protein eL39-like 5",
  "term_id": "GO:0003735",
  "term_label": "structural constituent of ribosome",
  "gene_symbol": "RPL39P5",
  "gene": "UniProtKB:Q59GN2"
}